cellular response to cAMP [GO:0071320] (biological process) Sources: GOC:mah Relationships: is a type of response to cAMP [GO:0051591]; is a type of cellular response to nitrogen compound [GO:1901699]; is a type of cellular response to oxygen-containing compound [GO:1901701] Definition: Any process that results in a change in state or activity of a cell (in terms of movement, secretion, enzyme production, gene expression, etc.) as a result of a cAMP (cyclic AMP, adenosine 3',5'-cyclophosphate) stimulus. Also known as: cellular response to 3',5' cAMP, cellular response to 3',5'-cAMP, cellular response to adenosine 3',5'-cyclophosphate, cellular response to cyclic AMP